{
  "gene_name": "Transmembrane protein 217",
  "term_id": "UNKNOWN:0001",
  "gene": "UniProtKB:Q8N7C4",
  "term_label": "Unknown molecular function",
  "gene_symbol": "TMEM217"
}